{
  "term_id": "GO:0005516",
  "gene_name": "Ras GTPase-activating-like protein IQGAP3",
  "gene": "UniProtKB:Q86VI3",
  "gene_symbol": "IQGAP3",
  "term_label": "calmodulin binding"
}